{
  "term_label": "regulation of DNA-templated transcription",
  "gene_name": "Ribosomal protein S6 kinase alpha-5",
  "gene_symbol": "RPS6KA5",
  "gene": "UniProtKB:O75582",
  "term_id": "GO:0006355"
}